{
  "gene_name": "Myelin transcription factor 1-like protein",
  "gene": "UniProtKB:Q9UL68",
  "term_label": "Unknown biological process",
  "gene_symbol": "MYT1L",
  "term_id": "UNKNOWN:0002"
}